{
  "term_label": "Unknown biological process",
  "term_id": "UNKNOWN:0002",
  "gene": "UniProtKB:Q8N808",
  "gene_name": "Solute carrier family 35 member G3",
  "gene_symbol": "SLC35G3"
}